arabinan transmembrane transporter activity [GO:0042901] (molecular function) Sources: GOC:jl, GOC:mtg_transport, ISBN:0815340729 Relationships: is a type of polysaccharide transmembrane transporter activity [GO:0015159] Definition: Enables the transfer of an arabinan, a polysaccharide composed of arabinose residues, from one side of a membrane to the other.